carnitine-CoA ligase activity [GO:0051108] (molecular function) Relationships: is a type of CoA-ligase activity [GO:0016405]; is a type of acid-amino acid ligase activity [GO:0016881] Also known as: crotonobetaine/carnitine-CoA ligase activity, carnitine synthetase activity Definition: Catalysis of the reaction: D-carnitine + CoA + ATP = AMP + diphosphate + D-carnitinyl-CoA. Sources: MetaCyc:DCARNCOALIG-RXN